{
  "gene_name": "Ankyrin repeat domain-containing protein 42",
  "term_id": "GO:0051059",
  "gene_symbol": "ANKRD42",
  "gene": "UniProtKB:Q8N9B4",
  "term_label": "NF-kappaB binding"
}